{
  "term_label": "positive regulation of DNA repair",
  "gene_symbol": "EYA4",
  "gene_name": "Eyes absent homolog 4",
  "term_id": "GO:0045739",
  "gene": "UniProtKB:O95677"
}